{
  "term_id": "UNKNOWN:0001",
  "gene_name": "Transferrin receptor protein 2",
  "gene": "UniProtKB:Q9UP52",
  "gene_symbol": "TFR2",
  "term_label": "Unknown molecular function"
}